N-acylphosphatidylethanolamine-specific phospholipase D activity [GO:0070290] (molecular function) Also known as: N-acyl-phosphatidylethanolamine-specific phospholipase D activity, NAPE-specific phospholipase D activity Definition: Catalysis of the reaction: H2O + N-acyl-1,2-diacyl-sn-glycero-3-phosphoethanolamine (NAPE) = a 1,2-diacyl-sn-glycero-3-phosphate + an N-acylethanolamine (NAE) + H+. References: PMID:14634025, PMID:15878693 Sources: RHEA:33159 Relationships: is_a phospholipase activity [GO:0004620]; is a type of phosphoric diester hydrolase activity [GO:0008081]